{
  "term_label": "nucleus",
  "gene_name": "MRN complex-interacting protein",
  "gene_symbol": "MRNIP",
  "gene": "UniProtKB:Q6NTE8",
  "term_id": "GO:0005634"
}